{
  "gene_name": "Cancer_testis antigen 62",
  "term_label": "Unknown biological process",
  "gene_symbol": "CT62",
  "gene": "UniProtKB:P0C5K7",
  "term_id": "UNKNOWN:0002"
}